{
  "term_label": "adaptive thermogenesis",
  "gene_name": "N-fatty-acyl-amino acid synthase_hydrolase PM20D1",
  "gene_symbol": "PM20D1",
  "term_id": "GO:1990845",
  "gene": "UniProtKB:Q6GTS8"
}